{
  "term_label": "extracellular matrix structural constituent",
  "gene_symbol": "MUC5AC",
  "gene_name": "Mucin-5AC",
  "gene": "UniProtKB:P98088",
  "term_id": "GO:0005201"
}